sno(s)RNA processing [GO:0043144] (biological process) Definition: Any process involved in the conversion of a primary snoRNA family RNA transcript into a mature snoRNA (eukaryota) or sRNA (archaea). References: PMID:12773397 Sources: GOC:go_curators, GOC:krc Relationships: is a type of RNA processing [GO:0006396]; is a type of GO:0016074 Subtypes: intronic snoRNA processing [GO:0031070], sno(s)RNA 3'-end processing [GO:0031126], snoRNA splicing [GO:0034247], box C/D sno(s)RNA processing [GO:0034963], box H/ACA sno(s)RNA processing [GO:0034964], GO:0180031 Regulation: regulated by regulation of snoRNA processing [GO:1902796]; negatively regulated by negative regulation of snoRNA processing [GO:1902797]; positively regulated by positive regulation of snoRNA processing [GO:1902798]